{
  "term_id": "GO:0047429",
  "gene_symbol": "ASMTL",
  "term_label": "nucleoside triphosphate diphosphatase activity",
  "gene_name": "Probable bifunctional dTTP_UTP pyrophosphatase_methyltransferase protein",
  "gene": "UniProtKB:O95671"
}